{
  "gene": "UniProtKB:Q9BV35",
  "term_label": "ADP transport",
  "gene_name": "Mitochondrial adenyl nucleotide antiporter SLC25A23",
  "term_id": "GO:0015866",
  "gene_symbol": "SLC25A23"
}